{
  "term_id": "GO:0048245",
  "gene_name": "C-C motif chemokine 1",
  "gene_symbol": "CCL1",
  "term_label": "eosinophil chemotaxis",
  "gene": "UniProtKB:P22362"
}